negative regulation of timing of exogen [GO:0051889] (biological process) Definition: Any process that stops, prevents, or reduces the frequency, rate or extent of timing of exogen, the shedding phase of the hair cycle. Also known as: inhibition of exogen, down regulation of exogen, down-regulation of exogen, downregulation of exogen, negative regulation of exogen Relationships: is a type of negative regulation of hair follicle maturation [GO:0048817]; is a type of regulation of timing of exogen [GO:0051887]; negatively regulates exogen [GO:0042638] Sources: GOC:ai, GOC:pr